{
  "term_label": "nicotinate-nucleotide adenylyltransferase activity",
  "term_id": "GO:0004515",
  "gene": "UniProtKB:Q9HAN9",
  "gene_name": "Nicotinamide_nicotinic acid mononucleotide adenylyltransferase 1",
  "gene_symbol": "NMNAT1"
}